{
  "gene_name": "Equilibrative nucleoside transporter 1",
  "term_id": "GO:0005886",
  "gene": "UniProtKB:Q99808",
  "gene_symbol": "SLC29A1",
  "term_label": "plasma membrane"
}